brain-derived neurotrophic factor receptor binding [GO:0031546] (molecular function) Definition: Binding to a brain-derived neurotrophic factor receptor. Also known as: BDNF receptor binding, brain-derived neurotrophic factor ligand Relationships: is a type of neurotrophin receptor binding [GO:0005165] Sources: GOC:mah